FAD biosynthetic process [GO:0006747] (biological process) References: PMID:20822113 Sources: GOC:ai Relationships: is a type of FAD metabolic process [GO:0046443]; is a type of flavin adenine dinucleotide biosynthetic process [GO:0072388] Also known as: FAD anabolism, FAD biosynthesis, FAD formation, FAD synthesis, oxidized flavin adenine dinucleotide biosynthesis, oxidized flavin adenine dinucleotide biosynthetic process, oxidized flavin-adenine dinucleotide biosynthesis, oxidized flavin-adenine dinucleotide biosynthetic process Definition: The chemical reactions and pathways resulting in the formation of FAD, the oxidized form of flavin-adenine dinucleotide.